{
  "term_label": "sperm axoneme assembly",
  "gene_symbol": "CFAP206",
  "term_id": "GO:0007288",
  "gene": "UniProtKB:Q8IYR0",
  "gene_name": "Cilia- and flagella-associated protein 206"
}